radial microtubular system formation [GO:0010245] (biological process) Sources: GOC:syr Relationships: is a type of microtubule cytoskeleton organization [GO:0000226] Definition: Formation of radial microtubular systems during male meiotic cytokinesis in plants.